polycystin complex [GO:0002133] (cellular component) Relationships: is a type of protein-containing complex [GO:0032991] References: PMID:11901144 Sources: GOC:hjd Definition: A stable heterodimeric complex composed of polycystin-1 and polycystin-2. Note: Different forms of the complex differing in type of N-glycosylation of polycystin-1 can exist (endoglycosidase sensitive and endoglycosidase resistant).